{
  "term_id": "GO:0006631",
  "gene_symbol": "CPT1C",
  "gene": "UniProtKB:Q8TCG5",
  "term_label": "fatty acid metabolic process",
  "gene_name": "Carnitine O-palmitoyltransferase 1, brain isoform"
}